regulation of L-threonine import across plasma membrane [GO:1900926] (BP) Also known as: regulation of L-threonine import, regulation of L-threonine uptake Definition: Any process that modulates the frequency, rate or extent of L-threonine import into cell. Subtypes: negative regulation of L-threonine import across plasma membrane [GO:1900927], positive regulation of L-threonine import across plasma membrane [GO:1900928] Sources: GOC:TermGenie Relationships: is a type of regulation of amino acid import across plasma membrane [GO:0010958]; is a type of regulation of organic acid transport [GO:0032890]; regulates L-threonine import across plasma membrane [GO:1903807]